{
  "gene": "UniProtKB:Q4G0G2",
  "term_id": "UNKNOWN:0003",
  "gene_name": "Putative uncharacterized protein H1-10-AS1",
  "gene_symbol": "H1-10-AS1",
  "term_label": "Unknown cellular component"
}